{
  "term_id": "GO:0001669",
  "gene": "UniProtKB:Q7RTX7",
  "gene_name": "Cation channel sperm-associated protein 4",
  "gene_symbol": "CATSPER4",
  "term_label": "acrosomal vesicle"
}